{
  "term_label": "Unknown biological process",
  "term_id": "UNKNOWN:0002",
  "gene_name": "Ornithine decarboxylase antizyme 2",
  "gene_symbol": "OAZ2",
  "gene": "UniProtKB:O95190"
}